{
  "gene": "UniProtKB:Q9UBD5",
  "gene_symbol": "ORC3",
  "gene_name": "Origin recognition complex subunit 3",
  "term_id": "GO:0005656",
  "term_label": "nuclear pre-replicative complex"
}